{
  "term_label": "immunoglobulin mediated immune response",
  "gene": "UniProtKB:A0A075B7B8",
  "gene_symbol": "IGHV3OR16-12",
  "gene_name": "Immunoglobulin heavy variable 3_OR16-12 (non-functional) (Fragment)",
  "term_id": "GO:0016064"
}